{
  "gene_name": "Ubiquitin carboxyl-terminal hydrolase 16",
  "gene_symbol": "USP16",
  "gene": "UniProtKB:Q9Y5T5",
  "term_label": "Unknown molecular function",
  "term_id": "UNKNOWN:0001"
}